{
  "term_label": "regulation of alternative mRNA splicing, via spliceosome",
  "term_id": "GO:0000381",
  "gene": "UniProtKB:P51513",
  "gene_name": "RNA-binding protein Nova-1",
  "gene_symbol": "NOVA1"
}